{
  "gene": "UniProtKB:Q9NQX0",
  "gene_symbol": "PRDM6",
  "term_label": "nucleus",
  "term_id": "GO:0005634",
  "gene_name": "Putative histone-lysine N-methyltransferase PRDM6"
}